{
  "gene_name": "Meiosis regulator and mRNA stability factor 1",
  "gene_symbol": "MARF1",
  "gene": "UniProtKB:Q9Y4F3",
  "term_label": "cytoplasm",
  "term_id": "GO:0005737"
}